{
  "gene": "UniProtKB:Q9NSB2",
  "term_id": "GO:0030280",
  "gene_symbol": "KRT84",
  "gene_name": "Keratin, type II cuticular Hb4",
  "term_label": "structural constituent of skin epidermis"
}